{
  "term_label": "cytoplasm",
  "term_id": "GO:0005737",
  "gene": "UniProtKB:Q9NST1",
  "gene_symbol": "PNPLA3",
  "gene_name": "1-acylglycerol-3-phosphate O-acyltransferase PNPLA3"
}